{
  "gene_symbol": "TMEM126B",
  "gene_name": "Complex I assembly factor TMEM126B, mitochondrial",
  "gene": "UniProtKB:Q8IUX1",
  "term_label": "mitochondrial respiratory chain complex I assembly",
  "term_id": "GO:0032981"
}